lymphocyte activation involved in immune response [GO:0002285] (biological process) Subtypes: T cell activation involved in immune response [GO:0002286], B cell activation involved in immune response [GO:0002312], natural killer cell activation involved in immune response [GO:0002323], natural killer cell proliferation involved in immune response [GO:0002324], natural killer cell differentiation involved in immune response [GO:0002325] Sources: GOC:add, ISBN:0781735149 Also known as: lymphocyte activation during immune response Definition: A change in morphology and behavior of a lymphocyte resulting from exposure to a specific antigen, mitogen, cytokine, chemokine, cellular ligand, or soluble factor, leading to the initiation or perpetuation of an immune response. Relationships: is a type of GO:0002366; is a type of lymphocyte activation [GO:0046649]